malonyl-CoA methyltransferase activity [GO:0102130] (molecular function) Sources: GOC:pz, RHEA:17105 Definition: Catalysis of the reaction: S-adenosyl-L-methionine + a malonyl-[acp] = S-adenosyl-L-homocysteine + a malonyl-[acp] methyl ester. Relationships: is a type of methyltransferase activity [GO:0008168]